{
  "term_id": "UNKNOWN:0002",
  "gene_symbol": "LGALS16",
  "term_label": "Unknown biological process",
  "gene": "UniProtKB:A8MUM7",
  "gene_name": "Galectin-16"
}